interleukin-17 receptor activity [GO:0030368] (molecular function) Sources: GOC:add, GOC:jl, GOC:signaling Subtypes: interleukin-17A receptor activity [GO:0038174], interleukin-25 receptor activity [GO:0045507], interleukin-27 receptor activity [GO:0045509] Also known as: IL-17 receptor activity, IL-17R Definition: Combining with any member of the interleukin-17 family of cytokines and transmitting the signal from one side of the membrane to the other to initiate a change in cell activity. Relationships: is a type of GO:0004896; BFO_0000051 interleukin-17 binding [GO:0019975]